{
  "gene_name": "Potassium_sodium hyperpolarization-activated cyclic nucleotide-gated channel 1",
  "term_id": "GO:0098855",
  "gene": "UniProtKB:O60741",
  "term_label": "HCN channel complex",
  "gene_symbol": "HCN1"
}